{
  "term_label": "Unknown biological process",
  "term_id": "UNKNOWN:0002",
  "gene_name": "MAPK regulated corepressor interacting protein 2",
  "gene": "UniProtKB:Q9BUT9",
  "gene_symbol": "MCRIP2"
}